{
  "term_label": "membrane protein ectodomain proteolysis",
  "gene_symbol": "PSEN2",
  "gene": "UniProtKB:P49810",
  "gene_name": "Presenilin-2",
  "term_id": "GO:0006509"
}